{
  "gene_name": "Bardet-Biedl syndrome 10 protein",
  "gene_symbol": "BBS10",
  "gene": "UniProtKB:Q8TAM1",
  "term_id": "UNKNOWN:0001",
  "term_label": "Unknown molecular function"
}